{
  "term_label": "Unknown molecular function",
  "gene_symbol": "IGF2-AS",
  "gene": "UniProtKB:Q6U949",
  "gene_name": "Putative insulin-like growth factor 2 antisense gene protein",
  "term_id": "UNKNOWN:0001"
}